11-oxo-beta-amyrin biosynthetic process [GO:1902383] (biological process) Also known as: 11-oxo-beta-amyrin anabolism, 11-oxo-beta-amyrin biosynthesis, 11-oxo-beta-amyrin formation, 11-oxo-beta-amyrin synthesis Definition: The chemical reactions and pathways resulting in the formation of 11-oxo-beta-amyrin. References: PMID:22128119 Sources: GOC:TermGenie Relationships: is a type of pentacyclic triterpenoid biosynthetic process [GO:0019745]; is a type of ketone biosynthetic process [GO:0042181]